nucleoside monophosphate kinase activity [GO:0050145] (molecular function) Sources: RHEA:24036 Subtypes: AMP kinase activity [GO:0004017], GMP kinase activity [GO:0004385], UMP kinase activity [GO:0033862], GO:0036430 Also known as: nucleoside-phosphate kinase activity, ATP:nucleoside-phosphate phosphotransferase activity, NMP-kinase activity, nucleotide kinase activity Relationships: is a type of phosphotransferase activity, phosphate group as acceptor [GO:0016776]; is a type of GO:0019205; is part of GO:0046940 Definition: Catalysis of the reaction: a ribonucleoside 5'-phosphate + ATP = a ribonucleoside 5'-diphosphate + ADP.